enoyl-CoA hydratase activity [GO:0004300] (molecular function) Sources: EC:4.2.1.17 Also known as: 3-hydroxy-fatty acyl-CoA dehydratase, 3-hydroxyacyl-CoA dehydratase, short-chain enoyl-CoA hydratase activity, (3S)-3-hydroxyacyl-CoA hydro-lyase activity, 2-enoyl-CoA hydratase activity, 2-octenoyl coenzyme A hydrase activity, acyl coenzyme A hydrase activity, beta-hydroxyacid dehydrase activity, beta-hydroxyacyl-CoA dehydrase activity, enol-CoA hydratase activity, enoyl hydrase activity, unsaturated acyl-CoA hydratase activity Definition: Catalysis of the reaction: a 3-hydroxy-fatty acyl-CoA = a enoyl-CoA + H2O. This reaction usually occurs in the reverse direction, leading to the reduction of the double bound of enoyl-CoA in position 2 or 3. Specific reactions catalyzed include: a 4-saturated-(3S)-3-hydroxyacyl-CoA = a (3E)-enoyl-CoA + H2O and a (3S)-3-hydroxyacyl-CoA = a (2E)-enoyl-CoA + H2O. Relationships: is a type of hydro-lyase activity [GO:0016836] Subtypes: GO:0018812, 3-hydroxypropionyl-CoA dehydratase activity [GO:0043956]